{
  "gene": "UniProtKB:Q8NA92",
  "term_label": "Unknown biological process",
  "gene_name": "THAP domain-containing protein 8",
  "gene_symbol": "THAP8",
  "term_id": "UNKNOWN:0002"
}